positive regulation of cell-cell adhesion [GO:0022409] (BP) Subtypes: negative regulation of border follicle cell delamination [GO:0030712], GO:0033634, positive regulation of homotypic cell-cell adhesion [GO:0034112], positive regulation of heterotypic cell-cell adhesion [GO:0034116], positive regulation of calcium-dependent cell-cell adhesion [GO:0046587], GO:0051041, GO:1900735, positive regulation of leukocyte cell-cell adhesion [GO:1903039], positive regulation of homophilic cell adhesion [GO:1903387], positive regulation of epithelial cell-cell adhesion involved in epithelium migration [GO:1903683], positive regulation of cell-cell adhesion mediated by cadherin [GO:2000049] Sources: GOC:isa_complete Relationships: is a type of GO:0022407; is a type of GO:0045785; positively regulates GO:0098609 Definition: Any process that activates or increases the rate or extent of cell adhesion to another cell. Also known as: up regulation of cell-cell adhesion, up-regulation of cell-cell adhesion, upregulation of cell-cell adhesion, activation of cell-cell adhesion, stimulation of cell-cell adhesion